cycloheximide transmembrane transporter activity [GO:0015243] (molecular function) Definition: Enables the transfer of cycloheximide from one side of a membrane to the other. Cycloheximide is an antibiotic produced by Streptomyces which interferes with protein synthesis in eukaryotes. Subtypes: GO:0015309 Relationships: is a type of alcohol transmembrane transporter activity [GO:0015665]; is a type of amide transmembrane transporter activity [GO:0042887]; is part of cycloheximide transport [GO:0015901] Also known as: cycloheximide transporter activity Sources: ISBN:0198506732